{
  "gene_name": "Glutaredoxin-3",
  "term_id": "GO:0005829",
  "term_label": "cytosol",
  "gene": "UniProtKB:O76003",
  "gene_symbol": "GLRX3"
}